protoaphin-aglucone dehydratase (cyclizing) activity [GO:0047452] (molecular function) Also known as: protoaphin dehydratase (cyclizing), protoaphin dehydratase activity, protoaphin-aglucone hydro-lyase (cyclizing), protoaphin-aglucone hydro-lyase (cyclizing; xanthoaphin-forming) Sources: EC:4.2.1.73, RHEA:23876 Definition: Catalysis of the reaction: protoaphin aglucone = H2O + xanthoaphin. Relationships: is a type of hydro-lyase activity [GO:0016836]